positive regulation of hydrogen peroxide catabolic process [GO:1903285] (biological process) Definition: Any process that activates or increases the frequency, rate or extent of hydrogen peroxide catabolic process. References: PMID:23507046 Sources: GOC:PARL, GOC:TermGenie, GOC:bf, GO_REF:0000058 Also known as: positive regulation of H2O2 catabolic process, positive regulation of hydrogen peroxide breakdown, positive regulation of hydrogen peroxide catabolism, positive regulation of hydrogen peroxide degradation, up regulation of H2O2 catabolic process, up regulation of hydrogen peroxide breakdown, up regulation of hydrogen peroxide catabolic process, up regulation of hydrogen peroxide catabolism, up regulation of hydrogen peroxide degradation, up-regulation of H2O2 catabolic process, up-regulation of hydrogen peroxide breakdown, up-regulation of hydrogen peroxide catabolic process, up-regulation of hydrogen peroxide catabolism, up-regulation of hydrogen peroxide degradation, upregulation of H2O2 catabolic process, upregulation of hydrogen peroxide breakdown, upregulation of hydrogen peroxide catabolic process, upregulation of hydrogen peroxide catabolism, upregulation of hydrogen peroxide degradation, activation of H2O2 catabolic process, activation of hydrogen peroxide breakdown, activation of hydrogen peroxide catabolic process, activation of hydrogen peroxide catabolism, activation of hydrogen peroxide degradation, activation of H2O2 scavenging, activation of detoxification of H2O2, activation of detoxification of hydrogen peroxide, activation of hydrogen peroxide removal, activation of hydrogen peroxide scavenging, positive regulation of H2O2 scavenging, positive regulation of detoxification of H2O2, positive regulation of detoxification of hydrogen peroxide, positive regulation of hydrogen peroxide removal, positive regulation of hydrogen peroxide scavenging, up regulation of H2O2 scavenging, up regulation of detoxification of H2O2, up regulation of detoxification of hydrogen peroxide, up regulation of hydrogen peroxide removal, up regulation of hydrogen peroxide scavenging, up-regulation of H2O2 scavenging, up-regulation of detoxification of H2O2, up-regulation of detoxification of hydrogen peroxide, up-regulation of hydrogen peroxide removal, up-regulation of hydrogen peroxide scavenging, upregulation of H2O2 scavenging, upregulation of detoxification of H2O2, upregulation of detoxification of hydrogen peroxide, upregulation of hydrogen peroxide removal, upregulation of hydrogen peroxide scavenging Relationships: is_a GO:0009896; is a type of regulation of hydrogen peroxide catabolic process [GO:2000295]; is_a GO:2000379; positively regulates hydrogen peroxide catabolic process [GO:0042744]